{
  "term_id": "UNKNOWN:0001",
  "gene": "UniProtKB:Q8WXI3",
  "term_label": "Unknown molecular function",
  "gene_name": "Ankyrin repeat and SOCS box protein 10",
  "gene_symbol": "ASB10"
}